{
  "term_label": "synaptic transmission involved in micturition",
  "gene_symbol": "CHRNB4",
  "term_id": "GO:0060084",
  "gene_name": "Neuronal acetylcholine receptor subunit beta-4",
  "gene": "UniProtKB:P30926"
}